{
  "gene_symbol": "ZG16B",
  "gene_name": "Zymogen granule protein 16 homolog B",
  "term_id": "GO:0005615",
  "term_label": "extracellular space",
  "gene": "UniProtKB:Q96DA0"
}